{
  "gene_symbol": "GPR22",
  "term_label": "cellular response to hormone stimulus",
  "term_id": "GO:0032870",
  "gene": "UniProtKB:Q99680",
  "gene_name": "G-protein coupled receptor 22"
}